{
  "gene": "UniProtKB:Q7Z6J6",
  "gene_symbol": "FRMD5",
  "gene_name": "FERM domain-containing protein 5",
  "term_id": "GO:0031032",
  "term_label": "actomyosin structure organization"
}